{
  "gene_symbol": "CCL27",
  "gene": "UniProtKB:Q9Y4X3",
  "term_label": "neutrophil chemotaxis",
  "gene_name": "C-C motif chemokine 27",
  "term_id": "GO:0030593"
}